P2Y10 nucleotide receptor binding [GO:0031819] (molecular function) Relationships: is a type of G protein-coupled nucleotide receptor binding [GO:0031811] Also known as: P2Y10 nucleotide receptor ligand Definition: Binding to a P2Y10 nucleotide receptor. Sources: GOC:mah, GOC:nln